{
  "gene_name": "L-xylulose reductase",
  "term_id": "GO:0050038",
  "term_label": "L-xylulose reductase (NADPH) activity",
  "gene_symbol": "DCXR",
  "gene": "UniProtKB:Q7Z4W1"
}